{
  "term_label": "vacuolar acidification",
  "gene_symbol": "ATP6V0D1",
  "gene": "UniProtKB:P61421",
  "gene_name": "V-type proton ATPase subunit d 1",
  "term_id": "GO:0007035"
}